aspartate-tRNA(Asn) ligase activity [GO:0050560] (molecular function) Sources: EC:6.1.1.23, MetaCyc:6.1.1.23-RXN Relationships: is a type of GO:0004812 Also known as: aspartate-tRNAAsn ligase activity, L-aspartate:tRNAAsx ligase (AMP-forming), nondiscriminating aspartyl-tRNA synthetase activity Definition: Catalysis of the reaction: tRNA(Asx) + L-aspartate + ATP = aspartyl-tRNA(Asx) + diphosphate + AMP.